{
  "gene_name": "Potassium_sodium hyperpolarization-activated cyclic nucleotide-gated channel 3",
  "term_id": "GO:0035725",
  "gene": "UniProtKB:Q9P1Z3",
  "term_label": "sodium ion transmembrane transport",
  "gene_symbol": "HCN3"
}